{
  "gene_symbol": "DNAAF9",
  "gene_name": "Dynein axonemal assembly factor 9",
  "term_id": "UNKNOWN:0002",
  "gene": "UniProtKB:Q5TEA3",
  "term_label": "Unknown biological process"
}